{
  "gene_symbol": "SECISBP2",
  "term_label": "ribonucleoprotein complex binding",
  "term_id": "GO:0043021",
  "gene_name": "Selenocysteine insertion sequence-binding protein 2",
  "gene": "UniProtKB:Q96T21"
}